{
  "gene_name": "UPF0500 protein C1orf216",
  "gene": "UniProtKB:Q8TAB5",
  "term_label": "Unknown molecular function",
  "term_id": "UNKNOWN:0001",
  "gene_symbol": "C1orf216"
}